{
  "term_id": "GO:0031201",
  "gene": "UniProtKB:Q99747",
  "gene_symbol": "NAPG",
  "gene_name": "Gamma-soluble NSF attachment protein",
  "term_label": "SNARE complex"
}